tricaffeoyl spermidine:S-adenosyl-L-methionine O-methyltransferase activity [GO:0080078] (molecular function) Definition: Catalysis of the transfer of a methyl group from S-adenosyl-L-methionine to the oxygen atom of a tricaffeoyl spermidine molecule. References: PMID:19077165 Relationships: is a type of O-methyltransferase activity [GO:0008171]